{
  "term_id": "GO:0015031",
  "gene_name": "Receptor activity-modifying protein 2",
  "term_label": "protein transport",
  "gene_symbol": "RAMP2",
  "gene": "UniProtKB:O60895"
}